{
  "term_id": "GO:0046703",
  "gene_symbol": "CLEC2D",
  "term_label": "natural killer cell lectin-like receptor binding",
  "gene": "UniProtKB:Q9UHP7",
  "gene_name": "C-type lectin domain family 2 member D"
}